{
  "gene_name": "Proline and serine-rich protein 2",
  "gene_symbol": "PROSER2",
  "gene": "UniProtKB:Q86WR7",
  "term_label": "Unknown cellular component",
  "term_id": "UNKNOWN:0003"
}